{
  "gene_name": "Trace amine-associated receptor 2",
  "term_id": "GO:0005886",
  "gene": "UniProtKB:Q9P1P5",
  "term_label": "plasma membrane",
  "gene_symbol": "TAAR2"
}